{
  "term_label": "vacuole fusion",
  "gene": "UniProtKB:Q96JC1",
  "gene_name": "Vam6_Vps39-like protein",
  "term_id": "GO:0097576",
  "gene_symbol": "VPS39"
}